{
  "gene_symbol": "KCNAB1",
  "gene_name": "Voltage-gated potassium channel subunit beta-1",
  "gene": "UniProtKB:Q14722",
  "term_id": "GO:0044325",
  "term_label": "transmembrane transporter binding"
}